{
  "term_label": "Unknown molecular function",
  "gene_name": "Claudin domain-containing protein 2",
  "gene_symbol": "CLDND2",
  "term_id": "UNKNOWN:0001",
  "gene": "UniProtKB:Q8NHS1"
}